{
  "gene_symbol": "TSPY26P",
  "gene": "UniProtKB:Q9H489",
  "term_label": "Unknown biological process",
  "term_id": "UNKNOWN:0002",
  "gene_name": "Putative testis-specific Y-encoded-like protein 3"
}